{
  "gene_name": "Kinesin heavy chain isoform 5A",
  "term_label": "microtubule binding",
  "term_id": "GO:0008017",
  "gene": "UniProtKB:Q12840",
  "gene_symbol": "KIF5A"
}